sperm nuclear envelope removal [GO:0035040] (biological process) Relationships: is a type of nuclear membrane disassembly [GO:0051081]; is part of GO:0035039 Definition: Removal of the sperm nuclear envelope, allowing entry of maternal factors into the sperm nucleus. References: PMID:11735001 Sources: GOC:bf